{
  "term_id": "GO:0005886",
  "gene_symbol": "CD44",
  "gene_name": "CD44 antigen",
  "gene": "UniProtKB:P16070",
  "term_label": "plasma membrane"
}